{
  "term_label": "Unknown cellular component",
  "term_id": "UNKNOWN:0003",
  "gene_name": "Zinc finger protein 157",
  "gene_symbol": "ZNF157",
  "gene": "UniProtKB:P51786"
}